negative regulation of protein localization to actin cortical patch [GO:1904371] (biological process) References: PMID:18216290 Sources: GOC:TermGenie, GO_REF:0000058 Relationships: is a type of regulation of protein localization to actin cortical patch [GO:1904370]; is_a negative regulation of protein localization to cell cortex [GO:1904777]; negatively regulates GO:0044379 Also known as: down regulation of protein localisation to actin cortical patch, down regulation of protein localization to actin cortical patch, down-regulation of protein localisation to actin cortical patch, down-regulation of protein localization to actin cortical patch, downregulation of protein localisation to actin cortical patch, downregulation of protein localization to actin cortical patch, negative regulation of protein localisation to actin cortical patch, inhibition of protein localisation to actin cortical patch, inhibition of protein localization to actin cortical patch Definition: Any process that stops, prevents or reduces the frequency, rate or extent of protein localization to actin cortical patch.